{
  "term_id": "GO:0005634",
  "gene_symbol": "UBAP2L",
  "gene_name": "Ubiquitin-associated protein 2-like",
  "gene": "UniProtKB:Q14157",
  "term_label": "nucleus"
}